{
  "gene_name": "Olfactory receptor 1A1",
  "term_label": "signal transduction",
  "term_id": "GO:0007165",
  "gene": "UniProtKB:Q9P1Q5",
  "gene_symbol": "OR1A1"
}